RNA polymerase IV core binding [GO:0001048] (molecular function) Definition: Binding to RNA polymerase IV core enzyme, a multisubunit eukaryotic nuclear RNA polymerase found in plants and involved in siRNA production. Relationships: is_a GO:0043175 References: PMID:19110459 Sources: GOC:txnOH